{
  "gene_name": "La-related protein 7",
  "term_label": "RNA binding",
  "gene_symbol": "LARP7",
  "term_id": "GO:0003723",
  "gene": "UniProtKB:Q4G0J3"
}